muscle organ development [GO:0007517] (BP) Definition: The process whose specific outcome is the progression of the muscle over time, from its formation to the mature structure. The muscle is an organ consisting of a tissue made up of various elongated cells that are specialized to contract and thus to produce movement and mechanical work. Subtypes: visceral muscle development [GO:0007522], branchiomeric skeletal muscle development [GO:0014707], chordate pharyngeal muscle development [GO:0043282], skeletal muscle organ development [GO:0060538], nematode pharyngeal muscle development [GO:0160096] Relationships: is a type of GO:0048513; is a type of muscle structure development [GO:0061061] Regulation: regulated by GO:0048634; negatively regulated by negative regulation of muscle organ development [GO:0048635]; positively regulated by GO:0048636 Sources: GOC:jid, ISBN:0198506732